UDP-N-acetylmuramoylalanine-D-glutamate ligase activity [GO:0008764] (molecular function) Definition: Catalysis of the reaction: D-glutamate + ATP + UDP-N-acetylmuramoyl-L-alanine = ADP + 2 H+ + phosphate + UDP-N-acetylmuramoyl-L-alanyl-D-glutamate. Also known as: D-glutamate ligase activity, D-glutamate-adding enzyme activity, MurD synthetase activity, UDP-Mur-NAC-L-Ala:D-Glu ligase activity, UDP-N-acetylmuramoyl-L-alanine:glutamate ligase (ADP-forming), UDP-N-acetylmuramoyl-L-alanyl-D-glutamate synthetase activity, uridine diphospho-N-acetylmuramoylalanyl-D-glutamate synthetase activity Relationships: is a type of GO:0016881 Sources: RHEA:16429